carbohydrate mediated signaling [GO:0009756] (biological process) Relationships: is a type of GO:0007165; is part of GO:0071322 Subtypes: GO:0010182 Also known as: carbohydrate mediated signalling Sources: GOC:sm Definition: The series of molecular signals mediated by the detection of carbohydrate.